{
  "gene_symbol": "VLDLR",
  "term_label": "apolipoprotein binding",
  "gene_name": "Very low-density lipoprotein receptor",
  "gene": "UniProtKB:P98155",
  "term_id": "GO:0034185"
}